{
  "gene_name": "BAG family molecular chaperone regulator 1",
  "term_id": "GO:0016020",
  "gene": "UniProtKB:Q99933",
  "gene_symbol": "BAG1",
  "term_label": "membrane"
}